{
  "gene_symbol": "CCNE2",
  "gene_name": "G1_S-specific cyclin-E2",
  "term_id": "GO:0005634",
  "term_label": "nucleus",
  "gene": "UniProtKB:O96020"
}